imidazole-containing compound catabolic process [GO:0052805] (biological process) Sources: GOC:curators Relationships: is a type of GO:0009056; is a type of imidazole-containing compound metabolic process [GO:0052803] Subtypes: histamine catabolic process [GO:0001695], L-histidine catabolic process [GO:0006548], GO:0052804 Definition: The chemical reactions and pathways resulting in the breakdown of imidazoles, five-membered organic heterocycle containing two nitrogen atoms at positions 1 and 3, or any of its derivatives; compounds containing an imidazole skeleton. Also known as: imidazole breakdown, imidazole catabolism, imidazole degradation